{
  "term_id": "GO:0005876",
  "term_label": "spindle microtubule",
  "gene_symbol": "AURKB",
  "gene_name": "Aurora kinase B",
  "gene": "UniProtKB:Q96GD4"
}